{
  "gene_name": "Dipeptidyl aminopeptidase-like protein 6",
  "term_id": "GO:0008076",
  "term_label": "voltage-gated potassium channel complex",
  "gene": "UniProtKB:P42658",
  "gene_symbol": "DPP6"
}